{
  "gene": "UniProtKB:Q14980",
  "gene_name": "Nuclear mitotic apparatus protein 1",
  "gene_symbol": "NUMA1",
  "term_label": "centrosome",
  "term_id": "GO:0005813"
}